{
  "gene": "UniProtKB:Q5RKV6",
  "gene_name": "Exosome complex component MTR3",
  "gene_symbol": "EXOSC6",
  "term_id": "GO:0016075",
  "term_label": "rRNA catabolic process"
}